{
  "term_id": "GO:0005886",
  "gene_symbol": "OR51A4",
  "term_label": "plasma membrane",
  "gene": "UniProtKB:Q8NGJ6",
  "gene_name": "Olfactory receptor 51A4"
}